{
  "gene_symbol": "IQGAP1",
  "term_id": "GO:1903479",
  "gene": "UniProtKB:P46940",
  "gene_name": "Ras GTPase-activating-like protein IQGAP1",
  "term_label": "mitotic actomyosin contractile ring assembly actin filament organization"
}